{
  "term_id": "UNKNOWN:0001",
  "gene_symbol": "CDR2",
  "gene": "UniProtKB:Q01850",
  "gene_name": "Cerebellar degeneration-related protein 2",
  "term_label": "Unknown molecular function"
}